{
  "gene_symbol": "RGS17",
  "term_id": "GO:0009898",
  "gene_name": "Regulator of G-protein signaling 17",
  "gene": "UniProtKB:Q9UGC6",
  "term_label": "cytoplasmic side of plasma membrane"
}